{
  "term_id": "GO:0003924",
  "gene_symbol": "RAB43",
  "term_label": "GTPase activity",
  "gene": "UniProtKB:Q86YS6",
  "gene_name": "Ras-related protein Rab-43"
}